(1->4)-alpha-glucan metabolic process [GO:0070629] (biological process) Also known as: (1->4)-alpha-D-glucan metabolism, 1,4-alpha-D-glucan metabolism, 1,4-alpha-glucan metabolism, alpha-1,4 glucan metabolic process, alpha-1,4 glucan metabolism Subtypes: (1->4)-alpha-glucan biosynthetic process [GO:0070630] Sources: GOC:mah Definition: The chemical reactions and pathways involving (1->4)-alpha-glucans, compounds composed of glucose residues linked by (1->4)-alpha-D-glucosidic bonds. Relationships: is a type of alpha-glucan metabolic process [GO:0030978]